{
  "term_id": "GO:0005549",
  "gene": "UniProtKB:Q9UGF5",
  "gene_name": "Olfactory receptor 14J1",
  "term_label": "odorant binding",
  "gene_symbol": "OR14J1"
}